serine-ethanolaminephosphate phosphodiesterase activity [GO:0047387] (molecular function) Relationships: is a type of GO:0008081 Sources: EC:3.1.4.13, RHEA:17113 Definition: Catalysis of the reaction: H2O + serine phosphoethanolamine = H+ + phosphoethanolamine + serine. Also known as: SEP diesterase activity, serine ethanolamine phosphodiester phosphodiesterase activity, serine-phosphoethanolamine ethanolaminephosphohydrolase activity